{
  "gene_name": "Protein-arginine deiminase type-6",
  "gene_symbol": "PADI6",
  "term_id": "UNKNOWN:0002",
  "gene": "UniProtKB:Q6TGC4",
  "term_label": "Unknown biological process"
}